{
  "term_label": "plasma membrane",
  "gene_symbol": "SH2B3",
  "term_id": "GO:0005886",
  "gene_name": "SH2B adapter protein 3",
  "gene": "UniProtKB:Q9UQQ2"
}